{
  "gene_symbol": "ANKRD30B",
  "gene": "UniProtKB:Q9BXX2",
  "term_id": "UNKNOWN:0001",
  "gene_name": "Ankyrin repeat domain-containing protein 30B",
  "term_label": "Unknown molecular function"
}